{
  "term_id": "UNKNOWN:0003",
  "term_label": "Unknown cellular component",
  "gene_name": "Beta-mannosidase",
  "gene": "UniProtKB:O00462",
  "gene_symbol": "MANBA"
}